{
  "gene_name": "bMERB domain-containing protein 1",
  "gene_symbol": "BMERB1",
  "gene": "UniProtKB:Q96MC5",
  "term_label": "Unknown molecular function",
  "term_id": "UNKNOWN:0001"
}